dolichylphosphate-mannose phosphodiesterase activity [GO:0047398] (molecular function) Sources: EC:3.1.4.49, MetaCyc:3.1.4.49-RXN Relationships: is a type of phosphoric diester hydrolase activity [GO:0008081] Definition: Catalysis of the reaction: dolichyl beta-D-mannosyl phosphate + H2O = dolichol-phosphate + mannose. Also known as: dolichyl-beta-D-mannosyl-phosphate dolichylphosphohydrolase activity, mannosylphosphodolichol phosphodiesterase activity